regulation of establishment of planar polarity [GO:0090175] (biological process) Relationships: is_a regulation of animal organ morphogenesis [GO:2000027]; regulates establishment of planar polarity [GO:0001736] Definition: Any process that modulates the rate, frequency or extent of the establishment of planar polarity, the coordinated organization of groups of cells in a tissue, such that they all orient to similar coordinates. Sources: GOC:ascb_2009, GOC:dph, GOC:tb Subtypes: regulation of establishment of planar polarity involved in neural tube closure [GO:0090178]